{
  "gene_symbol": "DND1",
  "gene": "UniProtKB:Q8IYX4",
  "term_id": "GO:0060965",
  "gene_name": "Dead end protein homolog 1",
  "term_label": "negative regulation of miRNA-mediated gene silencing"
}